{
  "gene_symbol": "CDK5R2",
  "gene_name": "Cyclin-dependent kinase 5 activator 2",
  "term_id": "GO:0019901",
  "term_label": "protein kinase binding",
  "gene": "UniProtKB:Q13319"
}